{
  "term_id": "GO:0038023",
  "gene_name": "Integrin alpha-2",
  "term_label": "signaling receptor activity",
  "gene_symbol": "ITGA2",
  "gene": "UniProtKB:P17301"
}